{
  "term_label": "RNA binding",
  "gene_name": "Exosome complex component RRP40",
  "gene_symbol": "EXOSC3",
  "term_id": "GO:0003723",
  "gene": "UniProtKB:Q9NQT5"
}